carboxymethyloxysuccinate lyase activity [GO:0047772] (molecular function) Also known as: carboxymethyloxysuccinate glycolate-lyase (fumarate-forming), carboxymethyloxysuccinate glycolate-lyase activity Relationships: is a type of GO:0016835 Sources: EC:4.2.99.12, RHEA:12336 Definition: Catalysis of the reaction: carboxymethoxysuccinate = fumarate + glycolate.